demethylmacrocin O-methyltransferase activity [GO:0030770] (molecular function) Sources: EC:2.1.1.102, RHEA:17573 Definition: Catalysis of the reaction: S-adenosyl-L-methionine(1+) + demethylmacrocin = S-adenosyl-L-homocysteine + H+ + macrocin. Relationships: is_a S-adenosylmethionine-dependent methyltransferase activity [GO:0008757] Also known as: S-adenosyl-L-methionine:demethylmacrocin 2'''-O-methyltransferase activity, demethylmacrocin methyltransferase activity